{
  "gene": "UniProtKB:P52895",
  "gene_name": "Aldo-keto reductase family 1 member C2",
  "term_id": "GO:0042448",
  "gene_symbol": "AKR1C2",
  "term_label": "progesterone metabolic process"
}